post-embryonic hindlimb morphogenesis [GO:0035129] (biological process) Relationships: is a type of post-embryonic limb morphogenesis [GO:0035127]; is a type of hindlimb morphogenesis [GO:0035137] Sources: GOC:bf Definition: The process, occurring after embryonic development, by which the anatomical structures of the hindlimb are generated and organized.